regulation of ossification [GO:0030278] (biological process) Definition: Any process that modulates the frequency, rate or extent of ossification, the formation of bone or of a bony substance or the conversion of fibrous tissue or of cartilage into bone or a bony substance. Also known as: regulation of bone biosynthesis, regulation of bone formation Subtypes: negative regulation of ossification [GO:0030279], GO:0030500, GO:0045778 Relationships: is a type of regulation of multicellular organismal process [GO:0051239]; regulates ossification [GO:0001503] Sources: GOC:go_curators